{
  "gene_symbol": "PFDN5",
  "term_label": "RNA polymerase II core complex assembly",
  "gene": "UniProtKB:Q99471",
  "term_id": "GO:1990114",
  "gene_name": "Prefoldin subunit 5"
}